{
  "term_id": "GO:0003700",
  "term_label": "DNA-binding transcription factor activity",
  "gene_symbol": "ZNF783",
  "gene": "UniProtKB:Q6ZMS7",
  "gene_name": "Zinc finger protein 783"
}